microtubule-based process [GO:0007017] (biological process) Relationships: is_a cellular process [GO:0009987] Sources: GOC:mah Regulation: regulated by regulation of microtubule-based process [GO:0032886] Subtypes: microtubule cytoskeleton organization [GO:0000226], microtubule-based movement [GO:0007018], oocyte microtubule cytoskeleton polarization [GO:0008103], GO:0031023, GO:0032121, GO:0051231, spindle midzone assembly [GO:0051255], microtubule-based peroxisome localization [GO:0060152], GO:0099112 Definition: Any cellular process that depends upon or alters the microtubule cytoskeleton, that part of the cytoskeleton comprising microtubules and their associated proteins.